{
  "term_id": "GO:0031201",
  "gene": "UniProtKB:Q86Y82",
  "term_label": "SNARE complex",
  "gene_symbol": "STX12",
  "gene_name": "Syntaxin-12"
}